{
  "gene_symbol": "ZNF491",
  "gene_name": "Zinc finger protein 491",
  "term_label": "DNA-binding transcription factor activity, RNA polymerase II-specific",
  "gene": "UniProtKB:Q8N8L2",
  "term_id": "GO:0000981"
}